{
  "gene_symbol": "PAK3",
  "gene": "UniProtKB:O75914",
  "gene_name": "Serine_threonine-protein kinase PAK 3",
  "term_id": "GO:0035556",
  "term_label": "intracellular signal transduction"
}